condensed chromosome, centromeric region [GO:0000779] (cellular component) Sources: GOC:elh, GOC:kmv Definition: The region of a condensed chromosome that includes the centromere and associated proteins, including the kinetochore. In monocentric chromosomes, this region corresponds to a single area of the chromosome, whereas in holocentric chromosomes, it is evenly distributed along the chromosome. Relationships: is a type of GO:0000775; is part of condensed chromosome [GO:0000793] Note: Note that this term can be used in place of the obsolete cellular component term 'centromere ; GO:0005698'. Use with caution because this term refers to a specific region of the chromosome and not a protein complex. Also known as: condensed chromosome, centric region, condensed nuclear chromosome, centromeric region, condensed chromosome, centromere, condensed chromosome, pericentric region